{
  "gene_name": "Semaphorin-3E",
  "gene_symbol": "SEMA3E",
  "gene": "UniProtKB:O15041",
  "term_label": "plasma membrane",
  "term_id": "GO:0005886"
}